{
  "term_label": "ISG15 transferase activity",
  "gene_name": "Ubiquitin-conjugating enzyme E2 E1",
  "term_id": "GO:0042296",
  "gene_symbol": "UBE2E1",
  "gene": "UniProtKB:P51965"
}